{
  "gene_name": "Oocyte-secreted protein 4A",
  "gene": "UniProtKB:A0A2R8YFL7",
  "gene_symbol": "OOSP4A",
  "term_id": "UNKNOWN:0003",
  "term_label": "Unknown cellular component"
}